{
  "term_id": "UNKNOWN:0001",
  "gene": "UniProtKB:P29083",
  "gene_name": "General transcription factor IIE subunit 1",
  "gene_symbol": "GTF2E1",
  "term_label": "Unknown molecular function"
}